regulation of systemic arterial blood pressure by renin-angiotensin [GO:0003081] (BP) Also known as: blood pressure regulation by renin-angiotensin Definition: The process in which renin-angiotensin modulates the force with which blood passes through the circulatory system. Subtypes: regulation of systemic arterial blood pressure by circulatory renin-angiotensin [GO:0001991], regulation of blood volume by renin-angiotensin [GO:0002016], GO:0002034, GO:0003086 Relationships: is a type of GO:0001990 Sources: GOC:mtg_cardio